{
  "gene_name": "S-adenosylmethionine-dependent nucleotide dehydratase RSAD2",
  "gene": "UniProtKB:Q8WXG1",
  "term_label": "defense response to virus",
  "term_id": "GO:0051607",
  "gene_symbol": "RSAD2"
}